{
  "gene_name": "Zinc transporter ZIP2",
  "gene_symbol": "SLC39A2",
  "term_id": "GO:0005385",
  "gene": "UniProtKB:Q9NP94",
  "term_label": "zinc ion transmembrane transporter activity"
}